{
  "term_id": "GO:0000922",
  "gene_symbol": "PLK5",
  "gene_name": "Inactive serine_threonine-protein kinase PLK5",
  "gene": "UniProtKB:Q496M5",
  "term_label": "spindle pole"
}